{
  "gene_name": "Notch homolog 2 N-terminal-like protein C",
  "term_label": "Unknown molecular function",
  "gene_symbol": "NOTCH2NLC",
  "gene": "UniProtKB:P0DPK4",
  "term_id": "UNKNOWN:0001"
}